{
  "term_id": "UNKNOWN:0003",
  "gene_symbol": "VWA5A",
  "gene": "UniProtKB:O00534",
  "gene_name": "von Willebrand factor A domain-containing protein 5A",
  "term_label": "Unknown cellular component"
}